{
  "gene_name": "Putative protein PLEKHA9",
  "gene_symbol": "PLEKHA8P1",
  "gene": "UniProtKB:O95397",
  "term_id": "GO:0035621",
  "term_label": "ER to Golgi ceramide transport"
}